{
  "gene_name": "Zinc finger protein 154",
  "term_label": "RNA polymerase II cis-regulatory region sequence-specific DNA binding",
  "gene": "UniProtKB:Q13106",
  "term_id": "GO:0000978",
  "gene_symbol": "ZNF154"
}